{
  "term_label": "cytoplasm",
  "gene": "UniProtKB:P60673",
  "gene_name": "Profilin-3",
  "gene_symbol": "PFN3",
  "term_id": "GO:0005737"
}